{
  "term_id": "UNKNOWN:0001",
  "gene_name": "Rho family-interacting cell polarization regulator 1",
  "term_label": "Unknown molecular function",
  "gene": "UniProtKB:Q6ZS17",
  "gene_symbol": "RIPOR1"
}